{
  "gene_symbol": "GPRASP2",
  "term_id": "GO:0001664",
  "gene": "UniProtKB:Q96D09",
  "gene_name": "G-protein coupled receptor-associated sorting protein 2",
  "term_label": "G protein-coupled receptor binding"
}